{
  "gene_name": "Small ribosomal subunit protein bS18m",
  "gene_symbol": "MRPS18C",
  "gene": "UniProtKB:Q9Y3D5",
  "term_id": "GO:0070181",
  "term_label": "small ribosomal subunit rRNA binding"
}